{
  "term_label": "Unknown biological process",
  "term_id": "UNKNOWN:0002",
  "gene_name": "ATP-binding cassette sub-family F member 3",
  "gene_symbol": "ABCF3",
  "gene": "UniProtKB:Q9NUQ8"
}